{
  "term_label": "axonemal A tubule inner sheath",
  "gene_symbol": "SPMIP11",
  "gene": "UniProtKB:A0A1B0GTD5",
  "gene_name": "Testis-expressed protein 49",
  "term_id": "GO:0160111"
}